{
  "gene": "UniProtKB:O15033",
  "gene_name": "Apoptosis-resistant E3 ubiquitin protein ligase 1",
  "gene_symbol": "AREL1",
  "term_id": "GO:0006511",
  "term_label": "ubiquitin-dependent protein catabolic process"
}